{
  "gene_name": "Adenylate cyclase type 2",
  "term_label": "cAMP biosynthetic process",
  "gene_symbol": "ADCY2",
  "gene": "UniProtKB:Q08462",
  "term_id": "GO:0006171"
}